{
  "term_label": "Unknown biological process",
  "gene_name": "Platelet-activating factor acetylhydrolase",
  "gene": "UniProtKB:Q13093",
  "term_id": "UNKNOWN:0002",
  "gene_symbol": "PLA2G7"
}